{
  "gene_symbol": "BTG4",
  "term_label": "Unknown molecular function",
  "gene": "UniProtKB:Q9NY30",
  "gene_name": "Protein BTG4",
  "term_id": "UNKNOWN:0001"
}